nucleoside diphosphate metabolic process [GO:0009132] (biological process) Definition: The chemical reactions and pathways involving a nucleoside diphosphate, a compound consisting of a nucleobase linked to a deoxyribose or ribose sugar esterified with diphosphate on the sugar. Also known as: nucleoside diphosphate metabolism Relationships: is a type of nucleoside phosphate metabolic process [GO:0006753] Sources: GOC:go_curators, ISBN:0198506732 Subtypes: nucleoside diphosphate biosynthetic process [GO:0009133], GO:0009134, GO:0009135, pyrimidine nucleoside diphosphate metabolic process [GO:0009138], ribonucleoside diphosphate metabolic process [GO:0009185]